{
  "gene_name": "Non-histone chromosomal protein HMG-14",
  "gene_symbol": "HMGN1",
  "term_label": "chromatin organization",
  "gene": "UniProtKB:P05114",
  "term_id": "GO:0006325"
}